{
  "gene_name": "L-amino-acid oxidase",
  "term_label": "L-amino-acid oxidase activity",
  "term_id": "GO:0001716",
  "gene_symbol": "IL4I1",
  "gene": "UniProtKB:Q96RQ9"
}